{
  "term_id": "UNKNOWN:0002",
  "gene": "UniProtKB:P0C7Q5",
  "term_label": "Unknown biological process",
  "gene_name": "Putative solute carrier family 35 member G4",
  "gene_symbol": "SLC35G4"
}